{
  "gene": "UniProtKB:Q6ZMJ2",
  "term_id": "GO:0006879",
  "term_label": "intracellular iron ion homeostasis",
  "gene_name": "Scavenger receptor class A member 5",
  "gene_symbol": "SCARA5"
}